{
  "gene": "UniProtKB:P41250",
  "term_label": "mitochondrion",
  "term_id": "GO:0005739",
  "gene_name": "Glycine--tRNA ligase",
  "gene_symbol": "GARS1"
}